{
  "term_label": "peptidyl-prolyl cis-trans isomerase activity",
  "gene": "UniProtKB:Q5VVH2",
  "gene_symbol": "FKBP1C",
  "term_id": "GO:0003755",
  "gene_name": "Peptidyl-prolyl cis-trans isomerase FKBP1C"
}